{
  "term_label": "cell surface",
  "gene_symbol": "UMOD",
  "term_id": "GO:0009986",
  "gene": "UniProtKB:P07911",
  "gene_name": "Uromodulin"
}